asperthecin catabolic process [GO:0036183] (biological process) Sources: GOC:di Relationships: is a type of GO:0019336; is a type of asperthecin metabolic process [GO:0036182]; is a type of ketone catabolic process [GO:0042182]; is a type of secondary metabolite catabolic process [GO:0090487] Also known as: asperthecin breakdown, asperthecin catabolism, asperthecin degradation Definition: The chemical reactions and pathways resulting in the breakdown of asperthecin, an anthraquinone pigment obtained from the mould Aspergillus nidulans.